{
  "term_label": "negative regulation of transcription by RNA polymerase II",
  "term_id": "GO:0000122",
  "gene": "UniProtKB:Q9Y618",
  "gene_symbol": "NCOR2",
  "gene_name": "Nuclear receptor corepressor 2"
}